{
  "gene_symbol": "CLDN34",
  "term_label": "plasma membrane",
  "gene": "UniProtKB:H7C241",
  "term_id": "GO:0005886",
  "gene_name": "Claudin-34"
}